{
  "gene": "UniProtKB:Q9NZN4",
  "gene_symbol": "EHD2",
  "gene_name": "EH domain-containing protein 2",
  "term_label": "endocytosis",
  "term_id": "GO:0006897"
}